regulation of protein transport [GO:0051223] (biological process) Definition: Any process that modulates the frequency, rate or extent of the directed movement of a protein into, out of or within a cell, or between cells, by means of some agent such as a transporter or pore. Subtypes: regulation of intracellular protein transport [GO:0033157], regulation of Golgi to plasma membrane protein transport [GO:0042996], GO:0050708, positive regulation of protein transport [GO:0051222], negative regulation of protein transport [GO:0051224], GO:0099145, regulation of lipoprotein transport [GO:0140075], GO:1904215, GO:1904589, regulation of ubiquitin-dependent endocytosis [GO:2000395] Sources: GOC:ai Relationships: is a type of GO:0051049; is a type of regulation of establishment of protein localization [GO:0070201]; regulates protein transport [GO:0015031]